virion binding [GO:0046790] (molecular function) Definition: Binding to a virion, either by binding to components of the capsid or the viral envelope. Sources: GOC:ai Relationships: is a type of protein binding [GO:0005515]